{
  "gene_name": "Regulator of G-protein signaling 11",
  "gene": "UniProtKB:O94810",
  "gene_symbol": "RGS11",
  "term_id": "GO:0043005",
  "term_label": "neuron projection"
}